{
  "gene": "UniProtKB:O15539",
  "term_label": "negative regulation of G protein-coupled receptor signaling pathway",
  "gene_name": "Regulator of G-protein signaling 5",
  "term_id": "GO:0045744",
  "gene_symbol": "RGS5"
}